post-embryonic foregut morphogenesis [GO:0048618] (biological process) Definition: The process in which the anatomical structures of the foregut are generated and organized, during the post-embryonic phase. Sources: GOC:jid, GOC:rc Relationships: is a type of GO:0009886; is part of GO:0007440